{
  "term_id": "GO:0031507",
  "gene": "UniProtKB:P45973",
  "gene_symbol": "CBX5",
  "term_label": "heterochromatin formation",
  "gene_name": "Chromobox protein homolog 5"
}